{
  "term_label": "Unknown biological process",
  "term_id": "UNKNOWN:0002",
  "gene_name": "INO80 complex subunit B",
  "gene_symbol": "INO80B",
  "gene": "UniProtKB:Q9C086"
}